regulation of TRAIL production [GO:0032679] (biological process) Subtypes: GO:0032719, positive regulation of TRAIL production [GO:0032759] Also known as: regulation of TRAIL biosynthetic process Relationships: is a type of regulation of tumor necrosis factor superfamily cytokine production [GO:1903555]; regulates TRAIL production [GO:0032639] Definition: Any process that modulates the frequency, rate, or extent of TRAIL production. Sources: GOC:mah